pyroptotic inflammatory response [GO:0070269] (BP) Also known as: pyroptosis Relationships: is a type of inflammatory response [GO:0006954] References: PMID:18846107, PMID:21760595, PMID:33883744 Definition: A gasdermin-dependent inflammatory response that is associated with the generation of pyrogenic mediators such as IL-1beta and IL-18. Gasdermins are activated by caspase-1 or caspase-4/11, or by certain granzymes. In some, but not all cells, it can lead to pyroptotic programmed cell death. Subtypes: pyroptotic cell death [GO:0141201] Regulation: positively regulated by positive regulation of pyroptotic inflammatory response [GO:0140639]; negatively regulated by negative regulation of pyroptotic inflammatory response [GO:0160028]